leukotriene-A4 hydrolase activity [GO:0004463] (molecular function) Relationships: is a type of GO:0016803 Definition: Catalysis of the reaction: H2O + leukotriene A(4) = leukotriene B(4). Sources: EC:3.3.2.6, RHEA:22324 Also known as: (7E,9E,11Z,14Z)-(5S,6S)-5,6-epoxyicosa-7,9,11,14-tetraenoate hydrolase activity, LTA-4 hydrolase activity, LTA4 hydrolase activity, LTA4H, leukotriene A(4) hydrolase activity, leukotriene A4 hydrolase activity Subtypes: GO:0008908